{
  "gene_symbol": "CLHC1",
  "gene": "UniProtKB:Q8NHS4",
  "term_label": "Unknown molecular function",
  "term_id": "UNKNOWN:0001",
  "gene_name": "Clathrin heavy chain linker domain-containing protein 1"
}